{
  "gene_name": "Ribosyldihydronicotinamide dehydrogenase [quinone]",
  "gene_symbol": "NQO2",
  "term_id": "UNKNOWN:0002",
  "term_label": "Unknown biological process",
  "gene": "UniProtKB:P16083"
}